{
  "gene_symbol": "LMNTD1",
  "term_label": "Unknown biological process",
  "gene_name": "Lamin tail domain-containing protein 1",
  "term_id": "UNKNOWN:0002",
  "gene": "UniProtKB:Q8N9Z9"
}